positive regulation of (R)-mevalonic acid biosynthetic process [GO:0106109] (biological process) References: PMID:24296663 Sources: GOC:BHF, GOC:BHF_miRNA, GOC:rph Relationships: is_a positive regulation of biosynthetic process [GO:0009891]; is a type of positive regulation of small molecule metabolic process [GO:0062013]; is a type of GO:0106107; positively regulates (R)-mevalonic acid biosynthetic process [GO:1901737] Definition: Any process that activates or increases the frequency, rate or extent of (R)-mevalonic acid biosynthetic process.